endocardial cushion development [GO:0003197] (biological process) Definition: The progression of a cardiac cushion over time, from its initial formation to the mature structure. The endocardial cushion is a specialized region of mesenchymal cells that will give rise to the heart septa and valves. Relationships: is a type of GO:0060485; is part of heart development [GO:0007507] Sources: GOC:mtg_heart